lateral part of cell [GO:0097574] (cellular component) Sources: GOC:pr Definition: The region of a polarized cell other than its tips or ends (in some cell types, one end may be called the apex and the other the base). For example, in a polarized epithelial cell, the lateral part includes the cell sides which interface adjacent cells. Subtypes: lateral part of motile cell [GO:0031255], lateral wall of outer hair cell [GO:0120249] Relationships: is a type of GO:0110165